{
  "gene_name": "NOP protein chaperone 1",
  "term_label": "Unknown cellular component",
  "gene_symbol": "NOPCHAP1",
  "term_id": "UNKNOWN:0003",
  "gene": "UniProtKB:Q8N5I9"
}